{
  "gene_symbol": "PABPC1L",
  "term_id": "GO:0005634",
  "term_label": "nucleus",
  "gene": "UniProtKB:Q4VXU2",
  "gene_name": "Polyadenylate-binding protein 1-like"
}